{
  "gene": "UniProtKB:Q17R89",
  "term_label": "GTPase activator activity",
  "gene_symbol": "ARHGAP44",
  "term_id": "GO:0005096",
  "gene_name": "Rho GTPase-activating protein 44"
}